{
  "term_label": "cytoplasm",
  "gene": "UniProtKB:Q9Y614",
  "term_id": "GO:0005737",
  "gene_symbol": "ACTL7B",
  "gene_name": "Actin-like protein 7B"
}